positive regulation of the force of heart contraction by epinephrine-norepinephrine [GO:0001997] (biological process) Definition: Any process that increases the force with which the cardiac muscles of the heart pump blood through the circulatory system as a result of the presence of epinephrine or norepinephrine in the bloodstream or released from the nerve endings. Relationships: is a type of positive regulation of the force of heart contraction by chemical signal [GO:0003099]; is part of GO:0003321 Also known as: increased force of heart contraction by adrenaline-noradrenaline, increased force of heart contraction by epinephrine-norepinephrine, increased strength of cardiac contraction by epinephrine-norepinephrine, increased inotropy by epinephrine-norepinephrine, positive regulation of heart contraction by adrenaline-noradrenaline, positive regulation of heart contraction by epinephrine-norepinephrine Sources: GOC:dph, GOC:mtg_cardio Subtypes: GO:0003089, GO:0003090